{
  "gene_symbol": "AAMP",
  "gene": "UniProtKB:Q13685",
  "term_label": "Unknown molecular function",
  "gene_name": "Angio-associated migratory cell protein",
  "term_id": "UNKNOWN:0001"
}